FAR/SIN/STRIPAK complex [GO:0090443] (cellular component) Also known as: SIN inhibitory phosphatase (SIP) complex, SIN inhibitory phosphatase complex, SIP complex, striatin interacting phosphatase and kinase complex, FAR complex, STRIPAK signalling complex Relationships: is a type of GO:0032991 Definition: A conserved protein phosphatase type 2A complex which contains a protein phosphatase type 2A, a protein phosphatase regulatory subunit, a striatin, an FHA domain protein and other subunits (at least six proteins). In fission yeast this complex negatively regulate the septation initiation network at the spindle pole body. References: PMID:21561862, PMID:22119525 Sources: GOC:vw